asialoglycoprotein receptor activity [GO:0004873] (molecular function) References: PMID:11278827, PMID:7624395 Sources: GOC:bf, Wikipedia:Asialoglycoprotein Definition: Receiving an asialoglycoprotein, and delivering the asialoglycoprotein into the cell via endocytosis. An asialoglycoprotein is a plasma glycoproteins from which the terminal sialic acid residue on their complex carbohydrate groups has been removed. The asialoglycoprotein receptor recognizes the terminal galactose and N-acetylgalactosamine units of the asialoglycoprotein, the receptor-ligand complex is internalized and transported to a sorting organelle where disassociation occurs before the receptor is recycled to the cell membrane. Relationships: is a type of cargo receptor activity [GO:0038024]